{
  "term_id": "GO:0019221",
  "gene": "UniProtKB:Q9NZH6",
  "gene_symbol": "IL37",
  "gene_name": "Interleukin-37",
  "term_label": "cytokine-mediated signaling pathway"
}